{
  "term_id": "GO:0004867",
  "gene_name": "Serpin B11",
  "gene": "UniProtKB:Q96P15",
  "term_label": "serine-type endopeptidase inhibitor activity",
  "gene_symbol": "SERPINB11"
}